protein-cysteine methyltransferase activity [GO:0106363] (MF) Definition: Catalysis of the reaction: L-cysteinyl-[protein] + S-adenosyl-L-methionine = H+ + S-adenosyl-L-homocysteine + S-methyl-L-cysteinyl-[protein]. References: PMID:21481189, PMID:22158122, PMID:24235145, PMID:25412445 Sources: GOC:sp, RHEA:66544 Also known as: protein cysteine methylase activity, protein cysteine methyltransferase activity Relationships: is a type of S-methyltransferase activity [GO:0008172]; is a type of GO:0008276; is a type of S-adenosylmethionine-dependent methyltransferase activity [GO:0008757]